negative regulation of (R)-mevalonic acid biosynthetic process [GO:0106108] (biological process) Definition: Any process that stops, prevents or reduces the frequency, rate or extent of (R)-mevalonic acid biosynthetic process. References: PMID:24296663 Sources: GOC:BHF, GOC:BHF_miRNA, GOC:rph Relationships: is a type of GO:0009890; is a type of negative regulation of small molecule metabolic process [GO:0062014]; is_a regulation of (R)-mevalonic acid biosynthetic process [GO:0106107]; negatively regulates (R)-mevalonic acid biosynthetic process [GO:1901737]